exit from host cell [GO:0035891] (biological process) Definition: The movement of an organism out of a cell of the host organism. The host is defined as the larger of the organisms involved in a symbiotic interaction. Also known as: host cell exit, ejection from host, ejection from host cell, exit from host Subtypes: viral release from host cell [GO:0019076], GO:0039674 References: PMID:19325115 Sources: GOC:bf, GOC:rs Relationships: is a type of biological process involved in interaction with host [GO:0051701]